{
  "gene_name": "DNA-directed RNA polymerase II subunit RPB11-a",
  "term_label": "transcription by RNA polymerase II",
  "gene": "UniProtKB:P52435",
  "gene_symbol": "POLR2J",
  "term_id": "GO:0006366"
}